T cell mediated cytotoxicity [GO:0001913] (biological process) Note: Note that either or both mechanisms mentioned in the definition may be used in this process. Note that both granule release and the engagement of death receptors on target cells result in the induction of apoptosis in the target cell. Note that both CD4 and CD8 positive T cells can mediate apoptosis of target cells, independently of their definition as 'helper' T cells or not. Also known as: T cell mediated apoptosis, T cell mediated cell death, T cell mediated cell killing, T lymphocyte mediated cytotoxicity, T-cell mediated apoptosis, T-cell mediated cell death, T-cell mediated cell killing, T-cell mediated cytotoxicity, T-lymphocyte mediated cytotoxicity, T cell mediated cytolysis Regulation: regulated by GO:0001914; RO_0002212 by negative regulation of T cell mediated cytotoxicity [GO:0001915]; positively regulated by positive regulation of T cell mediated cytotoxicity [GO:0001916] Definition: The directed killing of a target cell by a T cell through the release of granules containing cytotoxic mediators or through the engagement of death receptors. Subtypes: T cell mediated cytotoxicity directed against tumor cell target [GO:0002419] References: PMID:11911826 Sources: GOC:add, GOC:pr, ISBN:0781735149 Relationships: is a type of GO:0001909; is a type of T cell mediated immunity [GO:0002456]